{
  "gene_name": "Claudin-11",
  "gene_symbol": "CLDN11",
  "term_id": "GO:0005886",
  "term_label": "plasma membrane",
  "gene": "UniProtKB:O75508"
}